{
  "term_id": "GO:2000766",
  "gene": "UniProtKB:Q7Z5Q1",
  "gene_symbol": "CPEB2",
  "term_label": "negative regulation of cytoplasmic translation",
  "gene_name": "Cytoplasmic polyadenylation element-binding protein 2"
}